{
  "gene_name": "Ryanodine receptor 3",
  "term_label": "release of sequestered calcium ion into cytosol by sarcoplasmic reticulum",
  "gene": "UniProtKB:Q15413",
  "term_id": "GO:0014808",
  "gene_symbol": "RYR3"
}